{
  "gene": "UniProtKB:Q99598",
  "term_id": "GO:0005737",
  "term_label": "cytoplasm",
  "gene_symbol": "TSNAX",
  "gene_name": "Translin-associated protein X"
}